{
  "term_label": "extracellular matrix",
  "term_id": "GO:0031012",
  "gene_name": "Vitronectin",
  "gene": "UniProtKB:P04004",
  "gene_symbol": "VTN"
}